ribitol-5-phosphatase activity [GO:0110130] (molecular function) Relationships: is a type of phosphatase activity [GO:0016791] Definition: Catalysis of the reaction: ribitol-5-phosphate + H20 = ribitol + phosphate. References: PMID:30240188 Sources: GOC:rn